{
  "gene_name": "Glutathione peroxidase 3",
  "gene": "UniProtKB:P22352",
  "gene_symbol": "GPX3",
  "term_label": "glutathione peroxidase activity",
  "term_id": "GO:0004602"
}